{
  "term_label": "immunoglobulin complex",
  "term_id": "GO:0019814",
  "gene": "UniProtKB:P01705",
  "gene_name": "Immunoglobulin lambda variable 2-23",
  "gene_symbol": "IGLV2-23"
}